{
  "term_label": "Unknown biological process",
  "gene_symbol": "ALDH9A1",
  "gene_name": "4-trimethylaminobutyraldehyde dehydrogenase",
  "gene": "UniProtKB:P49189",
  "term_id": "UNKNOWN:0002"
}